{
  "gene_name": "Ras-related protein Rap-2a",
  "gene": "UniProtKB:P10114",
  "term_id": "GO:0030336",
  "term_label": "negative regulation of cell migration",
  "gene_symbol": "RAP2A"
}